{
  "term_id": "GO:0051011",
  "term_label": "microtubule minus-end binding",
  "gene": "UniProtKB:Q99871",
  "gene_symbol": "HAUS7",
  "gene_name": "HAUS augmin-like complex subunit 7"
}